regulation of adenosine receptor signaling pathway [GO:0060167] (biological process) Subtypes: positive regulation of adenosine receptor signaling pathway [GO:0060168], GO:0060169 Sources: GOC:dph Definition: Any process that modulates the frequency, rate or extent of the adenosine receptor signaling pathway. The adenosine receptor pathway is the series of molecular signals generated as a consequence of an adenosine receptor binding to one of its physiological ligands. Also known as: regulation of adenosine receptor signalling pathway Relationships: is a type of regulation of G protein-coupled receptor signaling pathway [GO:0008277]; regulates G protein-coupled adenosine receptor signaling pathway [GO:0001973]